{
  "term_id": "GO:0004930",
  "gene_name": "Adhesion G protein-coupled receptor G3",
  "term_label": "G protein-coupled receptor activity",
  "gene": "UniProtKB:Q86Y34",
  "gene_symbol": "ADGRG3"
}